DNA topoisomerase binding [GO:0044547] (molecular function) Definition: Binding to a DNA topoisomerase. Also known as: DNA topoisomerase I binding Sources: GOC:jl Relationships: is a type of enzyme binding [GO:0019899]